{
  "gene_symbol": "MT4",
  "gene_name": "Metallothionein-4",
  "gene": "UniProtKB:P47944",
  "term_label": "nucleus",
  "term_id": "GO:0005634"
}